response to bronchodilator [GO:0097366] (biological process) Definition: Any process that results in a change in state or activity of a cell or an organism (in terms of movement, secretion, enzyme production, gene expression, etc.) as a result of a bronchodilator stimulus. A bronchodilator is a chemical that causes an increase in the expansion of a bronchus or bronchial tubes. Also known as: response to bronchodilator agent, response to broncholytic agent Relationships: is a type of response to chemical [GO:0042221] Note: Note that this term is in the subset of terms that should not be used for direct manual annotation of gene products. It was created to be used for cross-referencing by other ontologies. Direct annotations to this term may be amended during annotation QC. Sources: GOC:hp